{
  "gene": "UniProtKB:Q92858",
  "gene_symbol": "ATOH1",
  "term_id": "GO:0070888",
  "term_label": "E-box binding",
  "gene_name": "Transcription factor ATOH1"
}